{
  "term_label": "DNA replication initiation",
  "term_id": "GO:0006270",
  "gene": "UniProtKB:P33993",
  "gene_symbol": "MCM7",
  "gene_name": "DNA replication licensing factor MCM7"
}